microtubule organizing center [GO:0005815] (cellular component) Relationships: is a type of cellular anatomical structure [GO:0110165]; is part of GO:0015630 References: PMID:17072892, PMID:17245416 Sources: GOC:vw, ISBN:0815316194, Wikipedia:Microtubule_organizing_center Definition: An intracellular structure that can catalyze gamma-tubulin-dependent microtubule nucleation and that can anchor microtubules by interacting with their minus ends, plus ends or sides. Also known as: MTOC, microtubule organising centre Subtypes: GO:0000923, centrosome [GO:0005813], spindle pole body [GO:0005816], GO:0031021, ciliary basal body [GO:0036064]